{
  "gene_symbol": "USP17L22",
  "gene_name": "Ubiquitin carboxyl-terminal hydrolase 17-like protein 22",
  "term_id": "GO:0004843",
  "term_label": "cysteine-type deubiquitinase activity",
  "gene": "UniProtKB:D6RA61"
}